GCN2-mediated signaling [GO:0140469] (biological process) Definition: A series of reactions in which a signal is passed on to downstream proteins within the cell via GCN2 (also known as EIF2AK4), an intracellular protein kinase that is activated by stress signals, such as amino acid starvation. References: PMID:27629041 Also known as: EIF2AK4-mediated signaling, regulation of eIF2 alpha phosphorylation by amino acid starvation Relationships: is a type of GO:0140467